{
  "gene_name": "Epidermal retinol dehydrogenase 2",
  "gene": "UniProtKB:Q8N3Y7",
  "term_label": "lipid droplet",
  "gene_symbol": "SDR16C5",
  "term_id": "GO:0005811"
}